{
  "gene_symbol": "PPIAL4H",
  "term_label": "cytoplasm",
  "gene_name": "Peptidyl-prolyl cis-trans isomerase A-like 4H",
  "gene": "UniProtKB:A0A075B767",
  "term_id": "GO:0005737"
}